{
  "gene": "UniProtKB:Q9NQS3",
  "gene_symbol": "NECTIN3",
  "term_id": "GO:0007156",
  "term_label": "homophilic cell-cell adhesion",
  "gene_name": "Nectin-3"
}